{
  "gene": "UniProtKB:Q5T197",
  "gene_name": "E3 ubiquitin-protein ligase DCST1",
  "term_id": "UNKNOWN:0001",
  "gene_symbol": "DCST1",
  "term_label": "Unknown molecular function"
}